{
  "term_id": "GO:0051011",
  "gene": "UniProtKB:Q96RT7",
  "gene_symbol": "TUBGCP6",
  "term_label": "microtubule minus-end binding",
  "gene_name": "Gamma-tubulin complex component 6"
}